{
  "gene_symbol": "H3-5",
  "term_id": "GO:0005634",
  "gene": "UniProtKB:Q6NXT2",
  "term_label": "nucleus",
  "gene_name": "Histone H3.3C"
}